{
  "term_label": "regulation of neurotransmitter secretion",
  "gene_symbol": "HCRT",
  "term_id": "GO:0046928",
  "gene_name": "Hypocretin neuropeptide precursor",
  "gene": "UniProtKB:O43612"
}